prostaglandin E receptor activity [GO:0004957] (molecular function) Sources: ISBN:0198506732 Also known as: PGE(2) receptor activity, PGE receptor activity Definition: Combining with prostaglandin E (PGE(2)) to initiate a change in cell activity. Relationships: is a type of GO:0004955